RZZ complex [GO:1990423] (cellular component) Definition: A kinetochore component required for both meiotic and mitotic spindle assembly checkpoints. References: PMID:12686595, PMID:15922598, PMID:20462495 Also known as: Rod-Zwilch-Zw10 complex Note: Example annotations for this term would be D. melanogaster mit(1)15 (Q9W4X9), rod and zwilch (Q9VA00). Relationships: is a type of protein-containing complex [GO:0032991]; BFO_0000050 GO:0000776